{
  "gene_name": "Extracellular sulfatase Sulf-2",
  "term_id": "GO:0010575",
  "term_label": "positive regulation of vascular endothelial growth factor production",
  "gene": "UniProtKB:Q8IWU5",
  "gene_symbol": "SULF2"
}